{
  "term_label": "Unknown biological process",
  "term_id": "UNKNOWN:0002",
  "gene": "UniProtKB:Q53H82",
  "gene_symbol": "LACTB2",
  "gene_name": "Endoribonuclease LACTB2"
}